{
  "gene_name": "Presenilin-2",
  "term_id": "GO:0070765",
  "term_label": "gamma-secretase complex",
  "gene_symbol": "PSEN2",
  "gene": "UniProtKB:P49810"
}